{
  "term_id": "GO:0005829",
  "gene": "UniProtKB:P52566",
  "gene_name": "Rho GDP-dissociation inhibitor 2",
  "gene_symbol": "ARHGDIB",
  "term_label": "cytosol"
}